{
  "gene_symbol": "KCTD2",
  "gene_name": "BTB_POZ domain-containing protein KCTD2",
  "term_id": "GO:0043161",
  "term_label": "proteasome-mediated ubiquitin-dependent protein catabolic process",
  "gene": "UniProtKB:Q14681"
}